{
  "gene_symbol": "USP17L13",
  "term_label": "regulation of protein stability",
  "gene_name": "Ubiquitin carboxyl-terminal hydrolase 17-like protein 13",
  "gene": "UniProtKB:C9JLJ4",
  "term_id": "GO:0031647"
}